{
  "term_id": "GO:0042995",
  "gene_symbol": "ACTN3",
  "term_label": "cell projection",
  "gene": "UniProtKB:Q08043",
  "gene_name": "Alpha-actinin-3"
}